{
  "term_label": "positive regulation of apoptotic process",
  "gene_name": "Serine_threonine-protein kinase 4",
  "gene": "UniProtKB:Q13043",
  "gene_symbol": "STK4",
  "term_id": "GO:0043065"
}